monosaccharide transmembrane transporter activity [GO:0015145] (molecular function) Definition: Enables the transfer of a monosaccharide from one side of a membrane to the other. Relationships: is a type of sugar transmembrane transporter activity [GO:0051119]; is part of monosaccharide transmembrane transport [GO:0015749] Subtypes: L-ascorbate:sodium symporter activity [GO:0008520], uronic acid transmembrane transporter activity [GO:0015133], pentose transmembrane transporter activity [GO:0015146], hexose transmembrane transporter activity [GO:0015149], L-ascorbic acid transmembrane transporter activity [GO:0015229], GO:0015407, 2-keto-3-deoxygluconate:proton symporter activity [GO:0015649] Sources: GOC:jl, GOC:mtg_transport, ISBN:0815340729